{
  "gene_name": "Apolipoprotein A-I",
  "term_label": "phospholipid binding",
  "gene": "UniProtKB:P02647",
  "term_id": "GO:0005543",
  "gene_symbol": "APOA1"
}